{
  "gene_name": "Golgi SNAP receptor complex member 1",
  "term_label": "SNARE complex",
  "gene": "UniProtKB:O95249",
  "gene_symbol": "GOSR1",
  "term_id": "GO:0031201"
}